symbiont-mediated evasion of recognition by host innate immune effector [GO:0141177] (biological process) References: PMID:19208801, PMID:33330873 Also known as: evasion of symbiont recognition by host innate immune effector Relationships: is a type of symbiont-mediated evasion of host innate immune response [GO:0141043] Subtypes: GO:0039699, GO:0099016, symbiont-mediated evasion of host restriction-modification system [GO:0099018], symbiont-mediated evasion of recognition by host complement [GO:0141178], symbiont-mediated evasion of recognition by host antimicrobial peptide [GO:0141179] Definition: A process by which a symbiont mitigates the effects of recognition by a host innate immune effector. Effectors have a direct activity against a symbiont and include complement, antimicrobial peptides, and bacterial restriction enzymes. The host is defined as the larger of the organisms involved in a symbiotic interaction.